catecholamine catabolic process [GO:0042424] (biological process) Definition: The chemical reactions and pathways resulting in the breakdown of any of a group of physiologically important biogenic amines that possess a catechol (3,4-dihydroxyphenyl) nucleus and are derivatives of 3,4-dihydroxyphenylethylamine. Relationships: is a type of catecholamine metabolic process [GO:0006584]; is a type of catechol-containing compound catabolic process [GO:0019614]; is a type of GO:0042402 Sources: GOC:jl, ISBN:0198506732 Also known as: catecholamine breakdown, catecholamine catabolism, catecholamine degradation Subtypes: epinephrine catabolic process [GO:0042419], dopamine catabolic process [GO:0042420], GO:0042422